{
  "gene_name": "Maestro heat-like repeat-containing protein family member 2B",
  "gene_symbol": "MROH2B",
  "term_label": "Unknown molecular function",
  "term_id": "UNKNOWN:0001",
  "gene": "UniProtKB:Q7Z745"
}